regulation of glycogen biosynthetic process [GO:0005979] (biological process) Sources: GOC:go_curators Also known as: regulation of glycogen anabolism, regulation of glycogen biosynthesis, regulation of glycogen formation, regulation of glycogen synthesis Subtypes: negative regulation of glycogen biosynthetic process [GO:0045719], positive regulation of glycogen biosynthetic process [GO:0045725] Relationships: is a type of regulation of glucan biosynthetic process [GO:0010962]; is a type of GO:0070873; regulates GO:0005978 Definition: Any process that modulates the frequency, rate or extent of the chemical reactions and pathways resulting in the formation of glycogen.